maintenance of protein location in cell [GO:0032507] (biological process) Sources: GOC:isa_complete, GOC:mah Definition: Any process in which a protein is maintained in a specific location within, or in the membrane of, a cell, and is prevented from moving elsewhere. Also known as: maintenance of protein localization in cell Subtypes: maintenance of protein location in cell cortex [GO:0032065], maintenance of protein location in mast cell secretory granule [GO:0033370], maintenance of protein location in T cell secretory granule [GO:0033377], GO:0045053, maintenance of protein localization in organelle [GO:0072595], maintenance of protein location in membrane [GO:0072658], maintenance of protein localization at cell tip [GO:0099017], GO:1990153 Relationships: is a type of maintenance of protein location [GO:0045185]; is a type of maintenance of location in cell [GO:0051651]